{
  "gene_name": "Dual specificity protein phosphatase 16",
  "term_label": "MAP kinase tyrosine/serine/threonine phosphatase activity",
  "gene": "UniProtKB:Q9BY84",
  "term_id": "GO:0017017",
  "gene_symbol": "DUSP16"
}